{
  "gene_symbol": "TANGO2",
  "gene": "UniProtKB:Q6ICL3",
  "term_id": "GO:0007030",
  "gene_name": "Transport and Golgi organization protein 2 homolog",
  "term_label": "Golgi organization"
}